regulation of endothelial tube morphogenesis [GO:1901509] (biological process) Relationships: is a type of regulation of morphogenesis of an epithelium [GO:1905330]; regulates endothelial tube morphogenesis [GO:0061154] Definition: Any process that modulates the frequency, rate or extent of endothelial tube morphogenesis. Sources: GOC:TermGenie, GOC:dph Subtypes: negative regulation of endothelial tube morphogenesis [GO:1905955], GO:1905956